{
  "gene_name": "Phosphatidate cytidylyltransferase, mitochondrial",
  "gene": "UniProtKB:Q96BW9",
  "gene_symbol": "TAMM41",
  "term_label": "phosphatidate cytidylyltransferase activity",
  "term_id": "GO:0004605"
}